{
  "gene_name": "Nuclear body protein SP140-like protein",
  "term_label": "regulation of transcription by RNA polymerase II",
  "term_id": "GO:0006357",
  "gene": "UniProtKB:Q9H930",
  "gene_symbol": "SP140L"
}